{
  "gene": "UniProtKB:O60304",
  "term_id": "GO:0000981",
  "term_label": "DNA-binding transcription factor activity, RNA polymerase II-specific",
  "gene_name": "Zinc finger protein 500",
  "gene_symbol": "ZNF500"
}